D-alanine transmembrane transport [GO:0042941] (biological process) Definition: The process in which D-alanine, the D-enantiomer of 2-aminopropanoic acid,  is transported across a lipid bilayer, from one side of a membrane to the other by means of some agent such as a transporter or pore. Relationships: is a type of GO:0003333; is a type of alanine transport [GO:0032328]; is_a D-amino acid transport [GO:0042940]; is a type of carboxylic acid transmembrane transport [GO:1905039] Subtypes: GO:0170048 Sources: GO:ew, GOC:jl, GOC:jsg, GOC:mah